positive regulation of sperm capacitation [GO:1902492] (biological process) Definition: Any process that activates or increases the frequency, rate or extent of sperm capacitation. References: PMID:22539676 Sources: GOC:TermGenie, GOC:hjd Also known as: up regulation of sperm capacitation, up-regulation of sperm capacitation, upregulation of sperm capacitation, activation of sperm capacitation, activation of sperm activation, positive regulation of sperm activation, up regulation of sperm activation, up-regulation of sperm activation, upregulation of sperm activation Relationships: is a type of positive regulation of multicellular organismal process [GO:0051240]; is a type of regulation of sperm capacitation [GO:1902490]; is a type of positive regulation of cell maturation [GO:1903431]; is a type of positive regulation of reproductive process [GO:2000243]; positively regulates sperm capacitation [GO:0048240]